{
  "term_id": "GO:0019957",
  "gene_symbol": "CXCR6",
  "gene": "UniProtKB:O00574",
  "term_label": "C-C chemokine binding",
  "gene_name": "C-X-C chemokine receptor type 6"
}